{
  "term_id": "GO:0046931",
  "gene_symbol": "PLEKHA7",
  "gene_name": "Pleckstrin homology domain-containing family A member 7",
  "gene": "UniProtKB:Q6IQ23",
  "term_label": "pore complex assembly"
}